{
  "gene_symbol": "NANS",
  "gene": "UniProtKB:Q9NR45",
  "term_label": "Unknown cellular component",
  "term_id": "UNKNOWN:0003",
  "gene_name": "Sialic acid synthase"
}